{
  "gene_symbol": "LRRC8B",
  "gene_name": "Volume-regulated anion channel subunit LRRC8B",
  "gene": "UniProtKB:Q6P9F7",
  "term_id": "GO:0098656",
  "term_label": "monoatomic anion transmembrane transport"
}